{
  "gene": "UniProtKB:B1AK53",
  "term_id": "GO:0005737",
  "gene_name": "Espin",
  "term_label": "cytoplasm",
  "gene_symbol": "ESPN"
}